tryptophan-independent indoleacetic acid biosynthetic process [GO:0009849] (biological process) Also known as: indoleacetic acid biosynthesis, tryptophan-independent, indoleacetic acid biosynthetic process, tryptophan-independent, tryptophan-independent IAA biosynthetic process, tryptophan-independent indoleacetic acid anabolism, tryptophan-independent indoleacetic acid biosynthesis, tryptophan-independent indoleacetic acid formation, tryptophan-independent indoleacetic acid synthesis Relationships: is a type of indoleacetic acid biosynthetic process [GO:0009684] References: PMID:10375566 Sources: GOC:go_curators, GOC:lm, GOC:lr Definition: The chemical reactions and pathways resulting in the formation of indoleacetic acid, independent of tryptophan.